pericanalicular vesicle [GO:0033675] (cellular component) References: PMID:15763347, PMID:9790571 Relationships: is a type of cytoplasmic vesicle [GO:0031410] Definition: A membrane-bounded vesicle found near the apical, or pericanalicular, membrane of a hepatocyte; contains proteins involved in bile salt transport and other fluid and solute transport processes.